{
  "term_id": "GO:0060294",
  "gene_name": "Dynein axonemal heavy chain 17",
  "gene_symbol": "DNAH17",
  "gene": "UniProtKB:Q9UFH2",
  "term_label": "cilium movement involved in cell motility"
}